positive regulation of cilium assembly [GO:0045724] (biological process) Subtypes: positive regulation of non-motile cilium assembly [GO:1902857], positive regulation of motile cilium assembly [GO:1905505] Definition: Any process that activates or increases the frequency, rate or extent of the formation of a cilium. Also known as: positive regulation of flagellum assembly, up regulation of cilium assembly, up-regulation of cilium assembly, upregulation of cilium assembly, activation of cilium assembly, stimulation of cilium assembly, positive regulation of flagellum biogenesis Relationships: is a type of positive regulation of plasma membrane bounded cell projection assembly [GO:0120034]; is a type of regulation of cilium assembly [GO:1902017]; is a type of positive regulation of organelle assembly [GO:1902117]; RO_0002213 cilium assembly [GO:0060271] Sources: GOC:cilia, GOC:go_curators